negative regulation of glutamate secretion, neurotransmission [GO:1903295] (biological process) Definition: Any process that stops, prevents or reduces the frequency, rate or extent of glutamate secretion, neurotransmission. Note: An example of this is Rab3gap1 in mouse (Q80UJ7) in PMID:16782817 inferred from mutant phenotype Relationships: is a type of negative regulation of glutamate secretion [GO:0014050]; is a type of GO:0046929; is a type of negative regulation of synaptic transmission, glutamatergic [GO:0051967]; is a type of regulation of glutamate secretion, neurotransmission [GO:1903294]; negatively regulates glutamate secretion, neurotransmission [GO:0061535] References: PMID:16782817 Sources: GOC:TermGenie, GO_REF:0000058 Also known as: down regulation of glutamate secretion, neurotransmission, down-regulation of glutamate secretion, neurotransmission, downregulation of glutamate secretion, neurotransmission, inhibition of glutamate secretion, neurotransmission